{
  "gene_symbol": "TRIM77",
  "term_id": "GO:0005737",
  "term_label": "cytoplasm",
  "gene": "UniProtKB:I1YAP6",
  "gene_name": "Tripartite motif-containing protein 77"
}